immunological synapse formation [GO:0001771] (biological process) Regulation: regulated by regulation of immunological synapse formation [GO:2000520]; negatively regulated by negative regulation of immunological synapse formation [GO:2000521]; positively regulated by positive regulation of immunological synapse formation [GO:2000522] Also known as: formation of immunological synapse Relationships: is a type of GO:0009988; is part of lymphocyte activation [GO:0046649] Definition: The formation of an area of close contact between a lymphocyte (T-, B-, or natural killer cell) and a target cell through the clustering of particular signaling and adhesion molecules and their associated membrane rafts on both the lymphocyte and target cell, which facilitates activation of the lymphocyte, transfer of membrane from the target cell to the lymphocyte, and in some situations killing of the target cell through release of secretory granules and/or death-pathway ligand-receptor interaction. References: PMID:11244041, PMID:11376330 Sources: GOC:mgi_curators